{
  "gene_symbol": "TMEM52B",
  "term_label": "Unknown molecular function",
  "gene": "UniProtKB:Q4KMG9",
  "gene_name": "Transmembrane protein 52B",
  "term_id": "UNKNOWN:0001"
}